{
  "term_id": "UNKNOWN:0002",
  "gene_name": "Uncharacterized protein C22orf31",
  "gene": "UniProtKB:O95567",
  "term_label": "Unknown biological process",
  "gene_symbol": "C22orf31"
}